{
  "term_id": "GO:0007520",
  "gene_symbol": "DOCK5",
  "gene_name": "Dedicator of cytokinesis protein 5",
  "gene": "UniProtKB:Q9H7D0",
  "term_label": "myoblast fusion"
}